{
  "term_id": "GO:0030316",
  "gene_name": "Macrophage colony-stimulating factor 1 receptor",
  "gene_symbol": "CSF1R",
  "gene": "UniProtKB:P07333",
  "term_label": "osteoclast differentiation"
}